anthocyanin 5-(6'''-hydroxycinnamoyltransferase) activity [GO:0047183] (molecular function) Relationships: is a type of acyltransferase activity, transferring groups other than amino-acyl groups [GO:0016747] Sources: EC:2.3.1.153, RHEA:15661 Definition: Catalysis of the reaction: (E)-4-coumaroyl-CoA + an anthocyanidin 3,5-di-O-beta-D-glucoside = an anthocyanidin 3-O-beta-D-glucoside 5-O-beta-D-[(6-O-(E)-4-coumaroyl)glucoside] + CoA. Caffeoyl-CoA can also act as an acyl donor. Also known as: anthocyanin 5-aromatic acyltransferase activity, hydroxycinnamoyl-CoA:anthocyanidin 3,5-diglucoside 5-O-glucoside-6'''-O-hydroxycinnamoyltransferase activity